Golgi lumen [GO:0005796] (cellular component) Subtypes: GO:0034469, trans-Golgi network transport vesicle lumen [GO:0098564] Definition: The volume enclosed by the membranes of any cisterna or subcompartment of the Golgi apparatus, including the cis- and trans-Golgi networks. Relationships: is a type of intracellular organelle lumen [GO:0070013]; is part of Golgi apparatus [GO:0005794] Also known as: Golgi apparatus lumen Sources: GOC:mah